{
  "gene": "UniProtKB:P62269",
  "gene_name": "Small ribosomal subunit protein uS13",
  "gene_symbol": "RPS18",
  "term_label": "structural constituent of ribosome",
  "term_id": "GO:0003735"
}